rhythmic inhibition [GO:0043180] (biological process) Relationships: is a type of rhythmic synaptic transmission [GO:0060024] Sources: GOC:go_curators Definition: Any process involved in the generation of rhythmic, synchronous inhibitory synaptic inputs in a neural circuit.